{
  "gene": "UniProtKB:P13535",
  "gene_symbol": "MYH8",
  "term_label": "myosin II complex",
  "gene_name": "Myosin-8",
  "term_id": "GO:0016460"
}